interleukin-3 receptor activity [GO:0004912] (MF) Definition: Combining with interleukin-3 and transmitting the signal from one side of the membrane to the other to initiate a change in cell activity. Sources: GOC:jl, GOC:signaling Also known as: IL-3 receptor activity, IL-3R Relationships: is a type of GO:0004896; is part of cellular response to interleukin-3 [GO:0036016]; is part of interleukin-3-mediated signaling pathway [GO:0038156]; has part interleukin-3 binding [GO:0019978]